{
  "gene": "UniProtKB:Q96KV6",
  "term_id": "GO:0050852",
  "gene_symbol": "BTN2A3P",
  "gene_name": "Putative butyrophilin subfamily 2 member A3",
  "term_label": "T cell receptor signaling pathway"
}